diplotene [GO:0000240] (biological process) Relationships: is a type of GO:0098764; is part of GO:0007128 Definition: The cell cycle phase which follows pachytene during prophase I of meiosis, during which the homologous chromosomes begin to separate and the synaptonemal complex dissolves. Sources: GOC:mtg_cell_cycle Note: Note that this term should not be used for direct annotation. If you are trying to make an annotation to x phase, it is likely that the correct annotation is 'regulation of x/y phase transition' or to a process which occurs during the reported phase (i.e mitotic DNA replication for mitotic S-phase). To capture the phase when a specific location or process is observed, the phase term can be used in an annotation extension (PMID:24885854) applied to a cellular component term (with the relation exists_during) or a biological process term (with the relation happens_during).